{
  "gene_symbol": "PEX16",
  "term_id": "UNKNOWN:0001",
  "gene": "UniProtKB:Q9Y5Y5",
  "gene_name": "Peroxisomal membrane protein PEX16",
  "term_label": "Unknown molecular function"
}